{
  "gene_symbol": "CRHR2",
  "term_label": "axon terminus",
  "gene": "UniProtKB:Q13324",
  "term_id": "GO:0043679",
  "gene_name": "Corticotropin-releasing factor receptor 2"
}